{
  "gene": "UniProtKB:Q9Y2L8",
  "gene_symbol": "ZKSCAN5",
  "term_label": "regulation of transcription by RNA polymerase II",
  "gene_name": "Zinc finger protein with KRAB and SCAN domains 5",
  "term_id": "GO:0006357"
}